transmembrane actin-associated (TAN) line [GO:1990973] (cellular component) Relationships: is a type of intracellular membraneless organelle [GO:0043232] Definition: A linear array of nuclear envelope membrane proteins composed of nesprin-2G and SUN2, which couple the nucleus to moving actin cables, resulting in rearward nuclear transport (away from the leading edge). References: PMID:21173262 Sources: GOC:hjd Also known as: TAN line